{
  "term_label": "glial cell differentiation",
  "gene": "UniProtKB:Q9UJH8",
  "gene_symbol": "METRN",
  "gene_name": "Meteorin",
  "term_id": "GO:0010001"
}